regulation of telomere maintenance in response to DNA damage [GO:1904505] (biological process) References: PMID:22579284 Sources: GOC:BHF, GOC:BHF_telomere, GOC:TermGenie, GOC:nc, GO_REF:0000058 Relationships: is a type of GO:0032204; is_a regulation of cellular response to stress [GO:0080135]; regulates GO:0043247 Also known as: regulation of DNA damage response, telomere maintenance Subtypes: negative regulation of telomere maintenance in response to DNA damage [GO:1904506], positive regulation of telomere maintenance in response to DNA damage [GO:1904507], GO:1905764 Definition: Any process that modulates the frequency, rate or extent of telomere maintenance in response to DNA damage.